{
  "gene_name": "Endosome_lysosome-associated apoptosis and autophagy regulator 1",
  "term_id": "GO:0005802",
  "term_label": "trans-Golgi network",
  "gene": "UniProtKB:Q6UXG2",
  "gene_symbol": "ELAPOR1"
}